{
  "term_id": "GO:0031145",
  "gene_name": "Anaphase-promoting complex subunit 5",
  "term_label": "anaphase-promoting complex-dependent catabolic process",
  "gene_symbol": "ANAPC5",
  "gene": "UniProtKB:Q9UJX4"
}